extrinsic component of presynaptic endocytic zone membrane [GO:0098894] (cellular component) Definition: The component of the presynaptic endocytic zone membrane consisting of gene products and protein complexes that are loosely bound to one of its surfaces, but not integrated into the hydrophobic region. Sources: GOC:autophagy, GOC:mf Relationships: is_a GO:0098888; is part of presynaptic endocytic zone membrane [GO:0098835]